{
  "term_id": "GO:0061631",
  "gene_symbol": "UBE2NL",
  "gene": "UniProtKB:Q5JXB2",
  "gene_name": "Putative ubiquitin-conjugating enzyme E2 N-like",
  "term_label": "ubiquitin conjugating enzyme activity"
}